{
  "gene": "UniProtKB:O75165",
  "term_id": "UNKNOWN:0001",
  "term_label": "Unknown molecular function",
  "gene_symbol": "DNAJC13",
  "gene_name": "DnaJ homolog subfamily C member 13"
}